mitochondrial tRNA thio-modification [GO:0070903] (biological process) Definition: The addition a sulfur atom to a nucleotide in a mitochondrial tRNA molecule. Subtypes: GO:1990799 Relationships: is a type of GO:0034227; is a type of mitochondrial tRNA modification [GO:0070900] Sources: GOC:mah, GOC:mcc